{
  "gene_name": "BCL-6 corepressor-like protein 1",
  "gene": "UniProtKB:Q5H9F3",
  "term_id": "GO:0003714",
  "term_label": "transcription corepressor activity",
  "gene_symbol": "BCORL1"
}